{
  "gene_name": "Long-chain fatty acid transport protein 1",
  "term_label": "long-chain fatty acid transmembrane transporter activity",
  "term_id": "GO:0005324",
  "gene": "UniProtKB:Q6PCB7",
  "gene_symbol": "SLC27A1"
}